{
  "term_label": "cytosolic large ribosomal subunit",
  "gene_symbol": "RPL5",
  "term_id": "GO:0022625",
  "gene": "UniProtKB:P46777",
  "gene_name": "Large ribosomal subunit protein uL18"
}